{
  "gene_symbol": "PDLIM1",
  "gene": "UniProtKB:O00151",
  "gene_name": "PDZ and LIM domain protein 1",
  "term_label": "actin binding",
  "term_id": "GO:0003779"
}